{
  "term_id": "GO:0008017",
  "gene_symbol": "MAP1S",
  "gene": "UniProtKB:Q66K74",
  "gene_name": "Microtubule-associated protein 1S",
  "term_label": "microtubule binding"
}